glycosulfatase activity [GO:0047966] (molecular function) Definition: Catalysis of the reaction: D-glucose 6-sulfate + H2O = D-glucose + H+ + sulfate. Sources: EC:3.1.6.3, RHEA:19145 Also known as: glycosulphatase activity, glucosulfatase activity, sugar-sulfate sulfohydrolase activity Relationships: is a type of sulfuric ester hydrolase activity [GO:0008484]